positive regulation of glucocorticoid biosynthetic process [GO:0031948] (BP) Definition: Any process that activates or increases the frequency, rate or extent of the chemical reactions and pathways resulting in the formation of glucocorticoids. Also known as: up regulation of glucocorticoid biosynthetic process, up-regulation of glucocorticoid biosynthetic process, upregulation of glucocorticoid biosynthetic process, activation of glucocorticoid biosynthetic process, stimulation of glucocorticoid biosynthetic process Relationships: is a type of GO:0031946; is a type of GO:0090031; positively regulates GO:0006704 Subtypes: positive regulation of cortisol biosynthetic process [GO:2000066] Sources: GOC:mah